{
  "gene_symbol": "FOXL1",
  "term_id": "GO:0030154",
  "term_label": "cell differentiation",
  "gene": "UniProtKB:Q12952",
  "gene_name": "Forkhead box protein L1"
}